{
  "gene_name": "Rho GTPase-activating protein 9",
  "gene_symbol": "ARHGAP9",
  "gene": "UniProtKB:Q9BRR9",
  "term_label": "GTPase activator activity",
  "term_id": "GO:0005096"
}